{
  "term_id": "GO:0005737",
  "gene": "UniProtKB:Q7Z569",
  "gene_symbol": "BRAP",
  "gene_name": "BRCA1-associated protein",
  "term_label": "cytoplasm"
}